{
  "gene_symbol": "COTL1",
  "gene_name": "Coactosin-like protein",
  "gene": "UniProtKB:Q14019",
  "term_id": "GO:0051015",
  "term_label": "actin filament binding"
}